EP4 subtype prostaglandin E2 receptor binding [GO:0031867] (molecular function) Definition: Binding to an EP4 subtype prostaglandin E2 receptor. Also known as: prostanoid EP4 receptor binding, EP4 subtype prostaglandin E2 receptor ligand Sources: GOC:mah, GOC:nln Relationships: is a type of prostanoid receptor binding [GO:0031862]